{
  "gene_symbol": "MT1X",
  "term_label": "metal ion binding",
  "term_id": "GO:0046872",
  "gene_name": "Metallothionein-1X",
  "gene": "UniProtKB:P80297"
}